nuclear DNA replication [GO:0033260] (biological process) Relationships: is a type of cell cycle DNA replication [GO:0044786]; BFO_0000066 GO:0005634 Sources: GOC:mtg_cell_cycle Subtypes: premeiotic DNA replication [GO:0006279], mitotic DNA replication [GO:1902969] Also known as: DNA replication involved in S phase, DNA replication involved in S-phase, nuclear cell cycle DNA replication, DNA replication during S phase Definition: The DNA-dependent DNA replication that occurs in the nucleus of eukaryotic organisms as part of the cell cycle. Regulation: positively regulated by GO:0010571; regulated by GO:0033262; negatively regulated by GO:1902576